{
  "gene_name": "NEDD8-conjugating enzyme Ubc12",
  "gene": "UniProtKB:P61081",
  "term_label": "cytosol",
  "term_id": "GO:0005829",
  "gene_symbol": "UBE2M"
}